{
  "gene_name": "Ras association domain-containing protein 5",
  "term_id": "GO:0005634",
  "gene": "UniProtKB:Q8WWW0",
  "term_label": "nucleus",
  "gene_symbol": "RASSF5"
}